{
  "term_id": "UNKNOWN:0002",
  "gene_symbol": "C10orf126",
  "gene": "UniProtKB:Q8N4M7",
  "term_label": "Unknown biological process",
  "gene_name": "Putative uncharacterized protein C10orf126"
}